negative regulation of intracellular transport of viral material [GO:1901253] (biological process) Definition: Any process that stops, prevents or reduces the frequency, rate or extent of intracellular transport of viral material. Also known as: down regulation of egress of virus within host cell, down regulation of movement of virus within host cell, down regulation of viral egress, down-regulation of egress of virus within host cell, down-regulation of movement of virus within host cell, down-regulation of viral egress, downregulation of egress of virus within host cell, downregulation of movement of virus within host cell, downregulation of viral egress, inhibition of movement of virus within host cell, inhibition of viral egress, negative regulation of movement of virus within host cell, negative regulation of viral egress, inhibition of egress of virus within host cell, negative regulation of egress of virus within host cell Relationships: is a type of regulation of intracellular transport of viral material [GO:1901252]; is a type of negative regulation of viral life cycle [GO:1903901]; negatively regulates intracellular transport of virus [GO:0075733] Sources: GOC:TermGenie, GOC:bf, GOC:jl